{
  "term_label": "negative regulation of appetite",
  "term_id": "GO:0032099",
  "gene_symbol": "CARTPT",
  "gene": "UniProtKB:Q16568",
  "gene_name": "Cocaine- and amphetamine-regulated transcript protein"
}